oligosaccharide biosynthetic process [GO:0009312] (biological process) Sources: ISBN:0198506732 Also known as: oligosaccharide anabolism, oligosaccharide biosynthesis, oligosaccharide formation, oligosaccharide synthesis Relationships: is_a GO:0009311; is a type of carbohydrate biosynthetic process [GO:0016051] Subtypes: GO:0009244, raffinose family oligosaccharide biosynthetic process [GO:0010325], GO:0046351, 6-alpha-maltosylglucose biosynthetic process [GO:0051680] Definition: The chemical reactions and pathways resulting in the formation of oligosaccharides, molecules with between two and (about) 20 monosaccharide residues connected by glycosidic linkages.